{
  "term_id": "UNKNOWN:0003",
  "term_label": "Unknown cellular component",
  "gene_name": "Tetratricopeptide repeat protein 13",
  "gene_symbol": "TTC13",
  "gene": "UniProtKB:Q8NBP0"
}